{
  "term_id": "GO:0000977",
  "term_label": "RNA polymerase II transcription regulatory region sequence-specific DNA binding",
  "gene_name": "Zinc finger protein 557",
  "gene_symbol": "ZNF557",
  "gene": "UniProtKB:Q8N988"
}